{
  "gene_symbol": "DLX3",
  "gene_name": "Homeobox protein DLX-3",
  "term_label": "epithelial cell differentiation",
  "term_id": "GO:0030855",
  "gene": "UniProtKB:O60479"
}